{
  "term_label": "plasma membrane",
  "gene_name": "Protocadherin beta-9",
  "gene": "UniProtKB:Q9Y5E1",
  "gene_symbol": "PCDHB9",
  "term_id": "GO:0005886"
}